{
  "term_label": "modulation of chemical synaptic transmission",
  "term_id": "GO:0050804",
  "gene": "UniProtKB:Q5JU85",
  "gene_symbol": "IQSEC2",
  "gene_name": "IQ motif and SEC7 domain-containing protein 2"
}